{
  "term_id": "GO:0016339",
  "gene": "UniProtKB:P55289",
  "term_label": "calcium-dependent cell-cell adhesion",
  "gene_symbol": "CDH12",
  "gene_name": "Cadherin-12"
}